{
  "term_label": "sensory perception of smell",
  "gene_name": "Putative olfactory receptor 8G2",
  "gene": "UniProtKB:Q6IF36",
  "gene_symbol": "OR8G2P",
  "term_id": "GO:0007608"
}